{
  "gene_name": "Beta-hexosaminidase subunit beta",
  "term_label": "ganglioside catabolic process",
  "gene": "UniProtKB:P07686",
  "gene_symbol": "HEXB",
  "term_id": "GO:0006689"
}